{
  "gene": "UniProtKB:Q5KU26",
  "term_id": "GO:0030198",
  "term_label": "extracellular matrix organization",
  "gene_symbol": "COLEC12",
  "gene_name": "Collectin-12"
}